fungiform papilla formation [GO:0061198] (biological process) Definition: The developmental process pertaining to the initial formation of a spongiform papilla from unspecified parts. The fungiform papilla is a mushroom-shaped papilla of the tongue. Relationships: is a type of anatomical structure formation involved in morphogenesis [GO:0048646]; is part of fungiform papilla morphogenesis [GO:0061197] Sources: GOC:dph